polyneuridine-aldehyde esterase activity [GO:0050529] (molecular function) Also known as: PNAE activity, polyneuridine aldehyde esterase activity, polyneuridine aldehyde hydrolase (decarboxylating) Sources: EC:3.1.1.78, RHEA:17501 Relationships: is a type of carboxylic ester hydrolase activity [GO:0052689] Definition: Catalysis of the reaction: H2O + polyneuridine aldehyde = 16-epivellosimine + CO2 + methanol.